{
  "gene_name": "Zinc finger protein 888",
  "gene": "UniProtKB:P0CJ79",
  "gene_symbol": "ZNF888",
  "term_label": "regulation of transcription by RNA polymerase II",
  "term_id": "GO:0006357"
}